{
  "gene_symbol": "H2AC19",
  "gene_name": "Histone H2A type 2-A",
  "gene": "UniProtKB:Q6FI13",
  "term_id": "GO:0000786",
  "term_label": "nucleosome"
}